{
  "gene_symbol": "KRTAP19-3",
  "gene_name": "Keratin-associated protein 19-3",
  "term_id": "UNKNOWN:0003",
  "term_label": "Unknown cellular component",
  "gene": "UniProtKB:Q7Z4W3"
}